{
  "gene": "UniProtKB:P57678",
  "term_id": "GO:0032797",
  "gene_symbol": "GEMIN4",
  "gene_name": "Gem-associated protein 4",
  "term_label": "SMN complex"
}